non-replicative DNA transposition [GO:0098038] (biological process) Relationships: is a type of DNA transposition [GO:0006313] References: PMID:2553270 Sources: GOC:bm Also known as: cut-and-paste transposition, non-replicative transposition, DNA-mediated Definition: Process by which a transposable element is excised from the donor site and integrated at the target site without replication of the element. Also referred to as cut-and-paste transposition.